{
  "gene_symbol": "DKC1",
  "term_id": "GO:0031120",
  "term_label": "snRNA pseudouridine synthesis",
  "gene_name": "H_ACA ribonucleoprotein complex subunit DKC1",
  "gene": "UniProtKB:O60832"
}